{
  "term_id": "GO:0005886",
  "gene_symbol": "DCHS2",
  "term_label": "plasma membrane",
  "gene": "UniProtKB:Q6V1P9",
  "gene_name": "Protocadherin-23"
}